diorcinol biosynthetic process [GO:1900572] (biological process) Also known as: diorcinol anabolism, diorcinol biosynthesis, diorcinol formation, diorcinol synthesis Definition: The chemical reactions and pathways resulting in the formation of diorcinol. Relationships: is a type of GO:0044550; is a type of phenol-containing compound biosynthetic process [GO:0046189]; is a type of diorcinol metabolic process [GO:1900570]; is a type of ether biosynthetic process [GO:1901503] Sources: GOC:TermGenie, GOC:di Regulation: regulated by GO:1900655; negatively regulated by negative regulation of diorcinol biosynthetic process [GO:1900656]; positively regulated by positive regulation of diorcinol biosynthetic process [GO:1900657]